{
  "term_id": "UNKNOWN:0002",
  "term_label": "Unknown biological process",
  "gene_symbol": "STMP1",
  "gene": "UniProtKB:E0CX11",
  "gene_name": "Short transmembrane mitochondrial protein 1"
}